{
  "gene": "UniProtKB:P25490",
  "term_id": "GO:0000978",
  "term_label": "RNA polymerase II cis-regulatory region sequence-specific DNA binding",
  "gene_name": "Transcriptional repressor protein YY1",
  "gene_symbol": "YY1"
}